{
  "gene_symbol": "LHX4",
  "gene": "UniProtKB:Q969G2",
  "gene_name": "LIM_homeobox protein Lhx4",
  "term_id": "GO:0005634",
  "term_label": "nucleus"
}